metanephric glomerular capillary formation [GO:0072277] (biological process) Definition: The process that gives rise to a metanephric glomerular capillary. This process pertains to the initial formation of a structure from unspecified parts. Relationships: is a type of glomerular capillary formation [GO:0072104]; is part of GO:0072276 Sources: GOC:mtg_kidney_jan10